{
  "gene_name": "Tripartite motif-containing protein 64",
  "term_id": "GO:0045087",
  "gene": "UniProtKB:A6NGJ6",
  "term_label": "innate immune response",
  "gene_symbol": "TRIM64"
}